thorny excrescence [GO:0097464] (cellular component) References: PMID:730852 Sources: NIF_Subcellular:nlx_467 Relationships: is a type of dendritic spine [GO:0043197] Definition: Large complex spine protruding from a dendrite. Each excrescence is formed by a cluster of spine heads.